{
  "gene_symbol": "E2F2",
  "gene_name": "Transcription factor E2F2",
  "gene": "UniProtKB:Q14209",
  "term_label": "RNA polymerase II transcription regulator complex",
  "term_id": "GO:0090575"
}